{
  "gene": "UniProtKB:P61221",
  "term_id": "GO:0005506",
  "gene_name": "ATP-binding cassette sub-family E member 1",
  "gene_symbol": "ABCE1",
  "term_label": "iron ion binding"
}